{
  "term_label": "carbohydrate metabolic process",
  "gene_symbol": "AMY1C",
  "term_id": "GO:0005975",
  "gene_name": "Alpha-amylase 1C",
  "gene": "UniProtKB:P0DTE8"
}